flavanone 4'-O-methyltransferase activity [GO:0102767] (molecular function) Definition: Catalysis of the reaction: (S)-naringenin + S-adenosyl-L-methionine = 2 H+ + ponciretin + S-adenosyl-L-homocysteine. Sources: EC:2.1.1.231, GOC:pz Relationships: is_a methyltransferase activity [GO:0008168]